homologous chromosome movement towards spindle pole in meiosis I anaphase [GO:0051758] (biological process) Definition: The directed movement of homologous chromosomes from the center of the spindle towards the spindle poles, mediated by the shortening of microtubules attached to the chromosomes, during meiosis I anaphase. Also known as: meiosis I, homologous chromosome movement towards spindle pole, homologous chromosome movement towards spindle pole during meiosis I Sources: GOC:ai Relationships: is a type of meiotic chromosome movement towards spindle pole [GO:0016344]; is part of homologous chromosome segregation [GO:0045143]